{
  "gene_symbol": "ALG9",
  "gene": "UniProtKB:Q9H6U8",
  "term_id": "GO:0005789",
  "gene_name": "Alpha-1,2-mannosyltransferase ALG9",
  "term_label": "endoplasmic reticulum membrane"
}